{
  "gene_name": "Heat shock protein beta-8",
  "term_id": "UNKNOWN:0001",
  "gene_symbol": "HSPB8",
  "term_label": "Unknown molecular function",
  "gene": "UniProtKB:Q9UJY1"
}